positive regulation of imaginal disc-derived wing vein specification [GO:0110108] (biological process) References: PMID:11861482 Sources: GOC:ha Relationships: is_a positive regulation of multicellular organismal process [GO:0051240]; is a type of GO:0110107; positively regulates imaginal disc-derived wing vein specification [GO:0007474] Definition: Any process that activates or increases the frequency, rate or extent of imaginal disc-derived wing vein specification.